anterior lateral line neuromast support cell differentiation [GO:0048906] (biological process) Relationships: is a type of neuromast support cell differentiation [GO:0048889]; is part of anterior lateral line neuromast development [GO:0048901] Definition: The process in which a relatively unspecialized cell acquires specialized features of an anterior lateral line neuromast support cell. Support cells are non-sensory cells of the neuromast that extend between the sensory hair cells from the basement membrane to the apical surface; they are surrounded by mantle cells. Sources: ISBN:0387968377